{
  "term_id": "UNKNOWN:0001",
  "gene_name": "Type III endosome membrane protein TEMP",
  "gene": "UniProtKB:Q8IVY1",
  "term_label": "Unknown molecular function",
  "gene_symbol": "C1orf210"
}